{
  "gene_symbol": "PAK3",
  "term_label": "cytoplasm",
  "term_id": "GO:0005737",
  "gene_name": "Serine_threonine-protein kinase PAK 3",
  "gene": "UniProtKB:O75914"
}